autonomic nervous system development [GO:0048483] (biological process) Definition: The process whose specific outcome is the progression of the autonomic nervous system over time, from its formation to the mature structure. The autonomic nervous system is composed of neurons that are not under conscious control, and is comprised of two antagonistic components, the sympathetic and parasympathetic nervous systems. The autonomic nervous system regulates key functions including the activity of the cardiac (heart) muscle, smooth muscles (e.g. of the gut), and glands. Sources: FMA:9905, GOC:jid, GOC:sr Subtypes: postganglionic parasympathetic fiber development [GO:0021784] Relationships: is a type of system development [GO:0048731]; is part of nervous system development [GO:0007399]